somatic motor neuron fate commitment [GO:0021917] (BP) Relationships: is a type of neuron fate commitment [GO:0048663]; is part of GO:0021523 Sources: GOC:cls, GOC:dgh, GOC:dph, GOC:jid, GO_REF:0000021 Definition: The commitment of unspecified motor neurons to specific motor neuron cell along the anterior-posterior axis of the spinal cord and their capacity to differentiate into specific motor neurons.